{
  "term_label": "extracellular space",
  "term_id": "GO:0005615",
  "gene": "UniProtKB:P04746",
  "gene_symbol": "AMY2A",
  "gene_name": "Pancreatic alpha-amylase"
}